{
  "gene_name": "Trafficking protein particle complex subunit 1",
  "term_id": "GO:0030008",
  "gene_symbol": "TRAPPC1",
  "gene": "UniProtKB:Q9Y5R8",
  "term_label": "TRAPP complex"
}